{
  "term_label": "extracellular region",
  "gene": "UniProtKB:Q9Y5W5",
  "gene_symbol": "WIF1",
  "gene_name": "Wnt inhibitory factor 1",
  "term_id": "GO:0005576"
}